{
  "term_label": "endocytosis",
  "gene_symbol": "HIP1",
  "gene": "UniProtKB:O00291",
  "gene_name": "Huntingtin-interacting protein 1",
  "term_id": "GO:0006897"
}